{
  "gene_symbol": "SLC6A18",
  "term_id": "UNKNOWN:0001",
  "gene": "UniProtKB:Q96N87",
  "gene_name": "Inactive sodium-dependent neutral amino acid transporter B(0)AT3",
  "term_label": "Unknown molecular function"
}